retina homeostasis [GO:0001895] (biological process) Relationships: is a type of tissue homeostasis [GO:0001894] Definition: A tissue homeostatic process involved in the maintenance of an internal equilibrium within the retina of the eye, including control of cellular proliferation and death and control of metabolic function. Subtypes: homeostasis of number of retina cells [GO:0048877], retina blood vessel maintenance [GO:0097601] References: PMID:15365173, PMID:15365178 Sources: GOC:add, GOC:dph, GOC:tb